{
  "term_label": "Unknown cellular component",
  "gene_symbol": "CFAP92",
  "gene_name": "Uncharacterized protein CFAP92",
  "gene": "UniProtKB:Q9ULG3",
  "term_id": "UNKNOWN:0003"
}